{
  "term_label": "vesicle docking involved in exocytosis",
  "term_id": "GO:0006904",
  "gene": "UniProtKB:O00186",
  "gene_symbol": "STXBP3",
  "gene_name": "Syntaxin-binding protein 3"
}